{
  "gene": "UniProtKB:P25024",
  "term_id": "GO:0006955",
  "gene_name": "C-X-C chemokine receptor type 1",
  "gene_symbol": "CXCR1",
  "term_label": "immune response"
}